{
  "gene": "UniProtKB:Q5H9M0",
  "gene_symbol": "PWWP3B",
  "term_label": "Unknown biological process",
  "gene_name": "PWWP domain-containing DNA repair factor 3B",
  "term_id": "UNKNOWN:0002"
}